{
  "gene": "UniProtKB:Q5T4F4",
  "term_id": "GO:0032584",
  "gene_symbol": "ZFYVE27",
  "term_label": "growth cone membrane",
  "gene_name": "Protrudin"
}